{
  "gene": "UniProtKB:Q8NHA8",
  "gene_symbol": "OR1F12P",
  "gene_name": "Putative olfactory receptor 1F12P",
  "term_label": "olfactory receptor activity",
  "term_id": "GO:0004984"
}